{
  "term_id": "GO:0034587",
  "gene": "UniProtKB:Q8NHU6",
  "gene_name": "Tudor domain-containing protein 7",
  "term_label": "piRNA processing",
  "gene_symbol": "TDRD7"
}